histamine secretion [GO:0001821] (biological process) Relationships: is a type of GO:0046903; is_a histamine transport [GO:0051608] Sources: GOC:mah, ISBN:0198506732, ISBN:0781735149 Definition: The regulated release of histamine by a cell or tissue. It is formed by decarboxylation of histidine and it acts through receptors in smooth muscle and in secretory systems. Subtypes: GO:0002441, GO:0061538